{
  "gene": "UniProtKB:P01270",
  "gene_symbol": "PTH",
  "term_id": "GO:0007267",
  "gene_name": "Parathyroid hormone",
  "term_label": "cell-cell signaling"
}